{
  "gene": "UniProtKB:O15204",
  "gene_symbol": "ADAMDEC1",
  "gene_name": "ADAM DEC1",
  "term_label": "metalloendopeptidase activity",
  "term_id": "GO:0004222"
}